{
  "gene": "UniProtKB:P0C6C1",
  "gene_name": "Ankyrin repeat domain-containing protein 34C",
  "term_id": "UNKNOWN:0001",
  "gene_symbol": "ANKRD34C",
  "term_label": "Unknown molecular function"
}